{
  "gene": "UniProtKB:Q9UBH6",
  "term_id": "GO:0006817",
  "gene_name": "Solute carrier family 53 member 1",
  "term_label": "phosphate ion transport",
  "gene_symbol": "XPR1"
}